{
  "gene_symbol": "SHH",
  "gene_name": "Sonic hedgehog protein",
  "term_label": "oligodendrocyte differentiation",
  "term_id": "GO:0048709",
  "gene": "UniProtKB:Q15465"
}